viral capsid [GO:0019028] (cellular component) Subtypes: helical viral capsid [GO:0019029], icosahedral viral capsid [GO:0019030] Sources: GOC:mtg_sensu, ISBN:0198506732 Relationships: is a type of virion component [GO:0044423] Definition: The protein coat that surrounds the infective nucleic acid in some virus particles. It comprises numerous regularly arranged subunits, or capsomeres.